{
  "term_id": "UNKNOWN:0003",
  "gene_name": "Zinc finger B-box domain-containing protein 1",
  "gene_symbol": "ZBBX",
  "gene": "UniProtKB:A8MT70",
  "term_label": "Unknown cellular component"
}